{
  "gene": "UniProtKB:A6NC78",
  "term_id": "GO:0005801",
  "gene_symbol": "GOLGA8IP",
  "gene_name": "Putative golgin subfamily A member 8I",
  "term_label": "cis-Golgi network"
}